{
  "gene": "UniProtKB:P46597",
  "term_id": "GO:0017096",
  "gene_symbol": "ASMT",
  "gene_name": "Acetylserotonin O-methyltransferase",
  "term_label": "acetylserotonin O-methyltransferase activity"
}